{
  "gene": "UniProtKB:P11464",
  "gene_symbol": "PSG1",
  "term_label": "Unknown molecular function",
  "term_id": "UNKNOWN:0001",
  "gene_name": "Pregnancy-specific beta-1-glycoprotein 1"
}